{
  "gene": "UniProtKB:Q7Z333",
  "gene_name": "Probable helicase senataxin",
  "term_id": "GO:0001147",
  "gene_symbol": "SETX",
  "term_label": "transcription termination site sequence-specific DNA binding"
}